exodeoxyribonuclease V activity [GO:0008854] (molecular function) Definition: Catalysis of the exonucleolytic cleavage (in the presence of ATP) in either 5' to 3' or 3' to 5' direction to yield 5'-phosphooligonucleotides. Also known as: E. coli exonuclease V activity, E. coli exonuclease V, Escherichia coli exonuclease V, RecBC deoxyribonuclease activity, exonuclease V activity, gene recBC DNase activity, gene recBC endoenzyme, gene recBCD enzymes Sources: EC:3.1.11.5 Relationships: is a type of DNA exonuclease activity, producing 5'-phosphomonoesters [GO:0016895]